{
  "term_id": "UNKNOWN:0002",
  "term_label": "Unknown biological process",
  "gene_symbol": "ZNF511",
  "gene_name": "Zinc finger protein 511",
  "gene": "UniProtKB:Q8NB15"
}